{
  "gene_name": "Probable G-protein coupled receptor 27",
  "term_id": "GO:0005886",
  "gene": "UniProtKB:Q9NS67",
  "term_label": "plasma membrane",
  "gene_symbol": "GPR27"
}